m7G(5')pppN diphosphatase complex [GO:0106095] (cellular component) Also known as: 7-methylguanosine-5'-triphospho-5'-polynucleotide 7-methylguanosine-5'-phosphohydrolase enzyme, DCS1 decapping scavenger complex, M(7)G(5')pppN pyrophosphatase enzyme, m7G(5')pppN diphosphatase enzyme, m7G(5')pppN pyrophosphatase enzyme Relationships: is a type of GO:1903293 References: PMID:22985415, PMID:26258763 Sources: GOC:lnp Definition: A homodimeric protein complex that catalyzes the reaction: 7-methylguanosine-5'-triphospho-5'-pholynucleotide + H20 = 7-methylguanosine-5'-phosphate + polynucleotide.